{
  "term_id": "GO:0005886",
  "term_label": "plasma membrane",
  "gene_symbol": "SPRED2",
  "gene": "UniProtKB:Q7Z698",
  "gene_name": "Sprouty-related, EVH1 domain-containing protein 2"
}